regulation of neutrophil mediated killing of fungus [GO:0070953] (BP) Subtypes: negative regulation of neutrophil mediated killing of fungus [GO:0070959], positive regulation of neutrophil mediated killing of fungus [GO:0070965] Sources: GOC:add, GOC:mah Definition: Any process that modulates the rate, frequency or extent of neutrophil mediated killing of a fungal cell, the directed killing of a fungal cell by a neutrophil. Relationships: is a type of regulation of neutrophil mediated killing of symbiont cell [GO:0070949]; is a type of GO:1900150; regulates neutrophil-mediated killing of fungus [GO:0070947]